positive regulation of endothelial cell activation [GO:1904989] (biological process) Also known as: up regulation of endothelial cell activation, up-regulation of endothelial cell activation, upregulation of endothelial cell activation, activation of endothelial cell activation References: PMID:24255059 Sources: GOC:BHF, GOC:BHF_miRNA, GOC:TermGenie, GOC:bc, GO_REF:0000058 Definition: Any process that activates or increases the frequency, rate or extent of endothelial cell activation. Relationships: is a type of positive regulation of cell activation [GO:0050867]; is a type of regulation of endothelial cell activation [GO:1904987]; RO_0002213 endothelial cell activation [GO:0042118]